{
  "gene_symbol": "UBXN10",
  "term_id": "GO:0043130",
  "gene": "UniProtKB:Q96LJ8",
  "gene_name": "UBX domain-containing protein 10",
  "term_label": "ubiquitin binding"
}